protein-arginine rhamnosyltransferase activity [GO:0106361] (molecular function) Relationships: is a type of glucosyltransferase activity [GO:0046527] References: PMID:25686373, PMID:26060278 Sources: GOC:sp, RHEA:66692 Definition: Catalysis of the reaction: dTDP-beta-L-rhamnose + L-arginyl-[protein] = dTDP + H+ + N(omega)-(L-rhamnosyl)-L-arginyl-[protein].